integrin binding involved in cell-matrix adhesion [GO:0098640] (molecular function) Definition: Any integrin binding that occurs as part of the process of cell-matrix adhesion. Relationships: is a type of integrin binding [GO:0005178]; is a type of GO:0098634 Sources: GOC:dos